{
  "gene": "UniProtKB:Q9BXX0",
  "term_id": "UNKNOWN:0002",
  "term_label": "Unknown biological process",
  "gene_symbol": "EMILIN2",
  "gene_name": "EMILIN-2"
}